{
  "gene": "UniProtKB:Q86YS3",
  "term_label": "endocytic vesicle",
  "gene_name": "Rab11 family-interacting protein 4",
  "gene_symbol": "RAB11FIP4",
  "term_id": "GO:0030139"
}